gamma-tubulin complex localization to mitotic spindle pole body [GO:1990735] (biological process) Definition: Any process in which a gamma-tubulin complex is transported to, or maintained in, a specific location at a mitotic spindle pole body. References: PMID:11080156 Sources: GOC:dos, GOC:mah Also known as: establishment and maintenance of gamma-tubulin complex localization to mitotic spindle pole body, gamma-tubulin complex localisation to mitotic spindle pole body, gamma-tubulin complex localization to mitotic SPB Relationships: is a type of GO:0033566 Subtypes: gamma-tubulin complex localization to nuclear side of mitotic spindle pole body [GO:0110120], gamma-tubulin complex localization to cytoplasmic side of mitotic spindle pole body [GO:0110121]